{
  "gene_name": "Transcription factor SOX-11",
  "gene": "UniProtKB:P35716",
  "term_id": "GO:0045944",
  "gene_symbol": "SOX11",
  "term_label": "positive regulation of transcription by RNA polymerase II"
}